{
  "term_label": "Unknown biological process",
  "gene": "UniProtKB:Q9H2H0",
  "term_id": "UNKNOWN:0002",
  "gene_name": "CXXC-type zinc finger protein 4",
  "gene_symbol": "CXXC4"
}